glandular epithelial cell development [GO:0002068] (biological process) Definition: The process whose specific outcome is the progression of a glandular epithelial cell over time, from its formation to the mature structure. A glandular epithelial cell is a columnar/cuboidal epithelial cell is a cell found in a two dimensional sheet with a free surface exposed to the lumen of a gland. Sources: GOC:dph Relationships: is a type of GO:0002066; BFO_0000050 glandular epithelial cell differentiation [GO:0002067] Subtypes: thyroid-stimulating hormone-secreting cell development [GO:0060130]